guanine metabolic process [GO:0046098] (biological process) Sources: GOC:go_curators Relationships: is a type of purine nucleobase metabolic process [GO:0006144] Subtypes: guanine catabolic process [GO:0006147], GMP catabolic process to guanine [GO:0006202], guanine biosynthetic process [GO:0046099] Definition: The chemical reactions and pathways involving guanine, 2-amino-6-hydroxypurine, a purine that is one of the five main bases found in nucleic acids and a component of a number of phosphorylated guanosine derivatives whose metabolic or regulatory functions are important. Also known as: guanine metabolism